beta-lactam antibiotic catabolic process [GO:0030655] (biological process) Definition: The chemical reactions and pathways resulting in the breakdown of a beta-lactam antibiotic, any member of a class of natural or semisynthetic antibiotics whose characteristic feature is a strained, four-membered beta-lactam ring. They include the penicillins and many of the cephalosporins. Sources: GOC:mah, ISBN:0198506732 Also known as: beta-lactam antibiotic breakdown, beta-lactam antibiotic catabolism, beta-lactam antibiotic degradation Relationships: is a type of antibiotic catabolic process [GO:0017001]; is a type of GO:0072340 Subtypes: penicillin catabolic process [GO:0042317], GO:1901117, GO:1901267, GO:1901768